{
  "gene": "UniProtKB:O75534",
  "gene_symbol": "CSDE1",
  "term_label": "CRD-mediated mRNA stabilization",
  "gene_name": "Cold shock domain-containing protein E1",
  "term_id": "GO:0070934"
}